oxidoreductase activity, acting on phosphorus or arsenic in donors, with a copper protein as acceptor [GO:0052882] (molecular function) Relationships: is a type of GO:0030613 Sources: GOC:jl Definition: Catalysis of an oxidation-reduction (redox) reaction in which a phosphorus- or arsenic-containing group acts as a hydrogen or electron donor and reduces a copper protein. Subtypes: arsenate reductase (azurin) activity [GO:0050611]